{
  "term_label": "extracellular space",
  "gene": "UniProtKB:Q9Y6L7",
  "gene_name": "Tolloid-like protein 2",
  "term_id": "GO:0005615",
  "gene_symbol": "TLL2"
}